{
  "term_id": "GO:0006081",
  "gene_name": "Aldehyde dehydrogenase, dimeric NADP-preferring",
  "gene": "UniProtKB:P30838",
  "term_label": "aldehyde metabolic process",
  "gene_symbol": "ALDH3A1"
}